{
  "term_id": "UNKNOWN:0001",
  "gene_name": "UBAP1-MVB12-associated (UMA)-domain containing protein 1",
  "gene_symbol": "UMAD1",
  "term_label": "Unknown molecular function",
  "gene": "UniProtKB:C9J7I0"
}